{
  "gene": "UniProtKB:O75746",
  "gene_name": "Electrogenic aspartate_glutamate antiporter SLC25A12, mitochondrial",
  "gene_symbol": "SLC25A12",
  "term_id": "GO:0043490",
  "term_label": "malate-aspartate shuttle"
}